{
  "term_id": "GO:0019838",
  "gene": "UniProtKB:Q02643",
  "gene_name": "Growth hormone-releasing hormone receptor",
  "gene_symbol": "GHRHR",
  "term_label": "growth factor binding"
}